{
  "gene": "UniProtKB:Q5EBL8",
  "gene_name": "PDZ domain-containing protein 11",
  "gene_symbol": "PDZD11",
  "term_id": "GO:0048489",
  "term_label": "synaptic vesicle transport"
}